{
  "gene_symbol": "OTUD7B",
  "gene": "UniProtKB:Q6GQQ9",
  "term_id": "GO:0043124",
  "gene_name": "OTU domain-containing protein 7B",
  "term_label": "negative regulation of canonical NF-kappaB signal transduction"
}